lumenal side of rough endoplasmic reticulum membrane [GO:0098555] (cellular component) Definition: The side (leaflet) of the rough endoplasmic reticulum membrane that faces the lumen. Relationships: is a type of lumenal side of endoplasmic reticulum membrane [GO:0098553]; is part of rough endoplasmic reticulum membrane [GO:0030867] Sources: GOC:ab, GOC:dos